{
  "term_id": "GO:0035627",
  "gene_name": "Phospholipid transfer protein",
  "term_label": "ceramide transport",
  "gene": "UniProtKB:P55058",
  "gene_symbol": "PLTP"
}